{
  "gene_name": "Armadillo repeat-containing X-linked protein 1",
  "term_id": "GO:0019896",
  "gene_symbol": "ARMCX1",
  "gene": "UniProtKB:Q9P291",
  "term_label": "axonal transport of mitochondrion"
}